{
  "gene_name": "Phosphoribosylformylglycinamidine synthase",
  "term_label": "cytoplasm",
  "gene_symbol": "PFAS",
  "term_id": "GO:0005737",
  "gene": "UniProtKB:O15067"
}